oxidoreductase activity, acting on a sulfur group of donors, disulfide as acceptor [GO:0016671] (molecular function) Also known as: oxidoreductase activity, acting on sulphur group of donors, disulphide as acceptor Relationships: is a type of oxidoreductase activity, acting on a sulfur group of donors [GO:0016667] Sources: GOC:jl Definition: Catalysis of an oxidation-reduction (redox) reaction in which a sulfur-containing group acts as a hydrogen or electron donor and reduces disulfide. Subtypes: phosphoadenylyl-sulfate reductase (thioredoxin) activity [GO:0004604], peptide-methionine (S)-S-oxide reductase activity [GO:0008113], GO:0019153, hydroperoxide reductase activity [GO:0032843], adenylyl-sulfate reductase (glutathione) activity [GO:0033741], GO:0033743, L-methionine (S)-S-oxide reductase activity [GO:0033744], L-methionine (R)-S-oxide reductase activity [GO:0033745], adenylyl-sulfate reductase (thioredoxin) activity [GO:0043866], GO:0047139, glutathione-CoA-glutathione transhydrogenase activity [GO:0047140], GO:0047141, enzyme-thiol transhydrogenase (glutathione-disulfide) activity [GO:0047142], protein-glutathione oxidoreductase (glutathione) activity [GO:0141049]